{
  "gene": "UniProtKB:Q9NPL8",
  "gene_name": "Complex I assembly factor TIMMDC1, mitochondrial",
  "term_label": "Unknown molecular function",
  "term_id": "UNKNOWN:0001",
  "gene_symbol": "TIMMDC1"
}